{
  "gene_name": "Azurocidin",
  "term_label": "serine-type endopeptidase activity",
  "term_id": "GO:0004252",
  "gene_symbol": "AZU1",
  "gene": "UniProtKB:P20160"
}